{
  "gene_name": "NADPH oxidase 3",
  "gene": "UniProtKB:Q9HBY0",
  "term_id": "GO:0016174",
  "gene_symbol": "NOX3",
  "term_label": "NAD(P)H oxidase H2O2-forming activity"
}